{
  "term_id": "UNKNOWN:0001",
  "gene_name": "Protein FAM240B",
  "term_label": "Unknown molecular function",
  "gene_symbol": "FAM240B",
  "gene": "UniProtKB:A0A1B0GVZ2"
}